petal structural organization [GO:0048452] (biological process) Relationships: is a type of floral organ structural organization [GO:0048450]; is part of petal morphogenesis [GO:0048446] Sources: GOC:jid Definition: The process that contributes to the act of creating the structural organization of the petal. This process pertains to the physical shaping of a rudimentary structure. Also known as: petal structural organisation